{
  "gene_name": "Toll_interleukin-1 receptor domain-containing adapter protein",
  "gene_symbol": "TIRAP",
  "gene": "UniProtKB:P58753",
  "term_id": "GO:0035663",
  "term_label": "Toll-like receptor 2 binding"
}